double layer follicle stage [GO:0048161] (BP) Relationships: is a type of GO:0022605 Also known as: mammalian oogenesis stage 4 Definition: The stage in oogenesis when a double layer of distinct follicle cells surrounds the oocyte. An example of this process is found in Mus musculus. Sources: GOC:jid, GOC:mtg_sensu, ISBN:0198542771